{
  "term_id": "UNKNOWN:0002",
  "gene_name": "Dual endothelin-1_angiotensin II receptor",
  "term_label": "Unknown biological process",
  "gene_symbol": "FBXW7-AS1",
  "gene": "UniProtKB:B0L3A2"
}